{
  "term_id": "UNKNOWN:0003",
  "gene": "UniProtKB:Q6ZTU2",
  "term_label": "Unknown cellular component",
  "gene_symbol": "EP400P1",
  "gene_name": "Putative EP400-like protein"
}